regulation of asexual sporulation [GO:0034305] (biological process) Definition: Any process that modulates the frequency, rate or extent of spore formation from the products of mitosis. Sources: GOC:mah Relationships: is_a regulation of sporulation [GO:0043937]; is a type of regulation of asexual reproduction [GO:1903664]; regulates asexual sporulation [GO:0030436] Also known as: regulation of asexual spore formation, regulation of mitotic spore formation, regulation of mitotic sporulation Subtypes: regulation of asexual sporulation resulting in formation of a cellular spore [GO:0043943], GO:0075306, regulation of oomycete sporangium development [GO:0075322]